sorbitol catabolic process [GO:0006062] (biological process) Definition: The chemical reactions and pathways resulting in the breakdown of sorbitol (D-glucitol), one of the ten stereoisomeric hexitols. It can be derived from glucose by reduction of the aldehyde group. Relationships: is_a sorbitol metabolic process [GO:0006060]; is_a hexitol catabolic process [GO:0019407] Sources: ISBN:0198506732 Also known as: sorbitol breakdown, sorbitol catabolism, sorbitol degradation